homocitrate synthase activity [GO:0004410] (molecular function) Relationships: is a type of GO:0046912 Definition: Catalysis of the reaction: 2-oxoglutarate + acetyl-CoA + H2O = CoA + H+ + homocitrate. Sources: RHEA:12929 Also known as: 2-hydroxybutane-1,2,4-tricarboxylate 2-oxoglutarate-lyase (CoA- acetylating) activity, 2-hydroxybutane-1,2,4-tricarboxylate 2-oxoglutarate-lyase (CoA-acetylating), acetyl-CoA:2-oxoglutarate C-acetyltransferase (thioester-hydrolysing, carboxymethyl forming), acetyl-coenzyme A:2-ketoglutarate C-acetyl transferase activity, homocitrate synthetase activity